{
  "gene_symbol": "CNTN5",
  "term_id": "GO:0098632",
  "gene_name": "Contactin-5",
  "gene": "UniProtKB:O94779",
  "term_label": "cell-cell adhesion mediator activity"
}